organelle transport along microtubule [GO:0072384] (biological process) Regulation: regulated by regulation of organelle transport along microtubule [GO:1902513] Subtypes: nuclear migration along microtubule [GO:0030473], lipid droplet transport along microtubule [GO:0031887], peroxisome transport along microtubule [GO:0036250], vesicle transport along microtubule [GO:0047496], mitochondrion transport along microtubule [GO:0047497], minus-end-directed organelle transport along microtubule [GO:0072385], plus-end-directed organelle transport along microtubule [GO:0072386] Also known as: microtubule-based organelle localization Definition: The directed movement of an organelle along a microtubule, mediated by motor proteins. This process begins with the attachment of an organelle to a microtubule, and ends when the organelle reaches its final destination. Sources: GOC:mah Relationships: is a type of transport along microtubule [GO:0010970]; is a type of establishment of organelle localization [GO:0051656]